{
  "term_label": "DNA-binding transcription activator activity, RNA polymerase II-specific",
  "gene_name": "Pre-B-cell leukemia transcription factor 2",
  "gene_symbol": "PBX2",
  "gene": "UniProtKB:P40425",
  "term_id": "GO:0001228"
}